{
  "gene": "UniProtKB:Q9UBS5",
  "term_id": "GO:0007214",
  "term_label": "gamma-aminobutyric acid signaling pathway",
  "gene_symbol": "GABBR1",
  "gene_name": "Gamma-aminobutyric acid type B receptor subunit 1"
}